{
  "term_label": "structural constituent of skin epidermis",
  "term_id": "GO:0030280",
  "gene_symbol": "KRT85",
  "gene": "UniProtKB:P78386",
  "gene_name": "Keratin, type II cuticular Hb5"
}